regulation of synapse assembly [GO:0051963] (BP) Subtypes: regulation of synaptic assembly at neuromuscular junction [GO:0008582], negative regulation of synapse assembly [GO:0051964], positive regulation of synapse assembly [GO:0051965], regulation of postsynapse assembly [GO:0150052], regulation of excitatory synapse assembly [GO:1904889], regulation of presynapse assembly [GO:1905606], GO:1905702 Definition: Any process that modulates the frequency, rate or extent of synapse assembly, the aggregation, arrangement and bonding together of a set of components to form a synapse. Also known as: regulation of synapse biogenesis, regulation of synaptogenesis Relationships: is a type of regulation of synapse organization [GO:0050807]; is a type of regulation of cell junction assembly [GO:1901888]; regulates GO:0007416 Sources: GOC:ai, GOC:pr